positive regulation of cytokinesis, actomyosin contractile ring assembly [GO:2000433] (biological process) Definition: Any process that activates or increases the frequency, rate or extent of cytokinesis, actomyosin contractile ring assembly. Subtypes: positive regulation of mitotic actomyosin contractile ring assembly [GO:1903501] Relationships: is a type of positive regulation of cytokinesis [GO:0032467]; is a type of positive regulation of cytoskeleton organization [GO:0051495]; is a type of regulation of cytokinesis, actomyosin contractile ring assembly [GO:2000431]; RO_0002213 actomyosin contractile ring assembly [GO:0000915] Sources: GOC:obol Also known as: positive regulation of contractile ring assembly